{
  "gene": "UniProtKB:Q14232",
  "term_id": "GO:0005851",
  "gene_symbol": "EIF2B1",
  "term_label": "eukaryotic translation initiation factor 2B complex",
  "gene_name": "Translation initiation factor eIF-2B subunit alpha"
}